regulation of endosome to plasma membrane protein transport [GO:1905749] (biological process) Subtypes: regulation of neurotransmitter receptor transport, endosome to postsynaptic membrane [GO:0099152], negative regulation of endosome to plasma membrane protein transport [GO:1905750], positive regulation of endosome to plasma membrane protein transport [GO:1905751] References: PMID:22869721 Sources: GOC:TermGenie, GO_REF:0000058 Relationships: is a type of regulation of intracellular protein transport [GO:0033157]; is_a regulation of protein localization to plasma membrane [GO:1903076]; is_a GO:2001135; regulates endosome to plasma membrane protein transport [GO:0099638] Definition: Any process that modulates the frequency, rate or extent of endosome to plasma membrane protein transport.